{
  "term_id": "GO:0042632",
  "gene_name": "Cytochrome P450 7A1",
  "gene": "UniProtKB:P22680",
  "term_label": "cholesterol homeostasis",
  "gene_symbol": "CYP7A1"
}